{
  "gene_name": "T cell receptor beta variable 6-6",
  "term_id": "UNKNOWN:0001",
  "gene_symbol": "TRBV6-6",
  "term_label": "Unknown molecular function",
  "gene": "UniProtKB:A0A0A6YYG2"
}